TDP metabolic process [GO:0046043] (biological process) Subtypes: TDP biosynthetic process [GO:0006232], GO:0006245 Definition: The chemical reactions and pathways involving TDP, ribosylthymine diphosphate. Relationships: is a type of pyrimidine ribonucleoside diphosphate metabolic process [GO:0009193]; is_a pyrimidine ribonucleotide metabolic process [GO:0009218] Sources: GOC:go_curators Also known as: TDP metabolism